RNA polymerase II transcription regulator complex [GO:0090575] (cellular component) Definition: A transcription factor complex that acts at a regulatory region of a gene transcribed by RNA polymerase II. Sources: GOC:tb Relationships: is_a transcription regulator complex [GO:0005667]; is a type of nuclear protein-containing complex [GO:0140513] Also known as: RNA polymerase II transcription factor complex Subtypes: transcription factor TFIIH core complex [GO:0000439], transcription factor TFIID complex [GO:0005669], GO:0005672, transcription factor TFIIE complex [GO:0005673], GO:0005674, transcription factor TFIIH holo complex [GO:0005675], ecdysone receptor holocomplex [GO:0008230], core-binding factor complex [GO:0016513], CCAAT-binding factor complex [GO:0016602], insulin control element activator complex [GO:0030232], GO:0030907, activin responsive factor complex [GO:0032444], transcription factor TFTC complex [GO:0033276], SBF transcription complex [GO:0033309], SMN-Gemin2 complex [GO:0034718], GO:0035189, transcription factor AP-1 complex [GO:0035976], CHOP-C/EBP complex [GO:0036488], Pi Mi complex [GO:0062071], SRF-myogenin-E12 complex [GO:0070514], ISGF3 complex [GO:0070721], core mediator complex [GO:0070847], transcription factor TFIIK complex [GO:0070985], heteromeric SMAD protein complex [GO:0071144], Myc-Max complex [GO:0071943], Pip2-Oaf1 complex [GO:0089716], M/G1 phase-specific MADS box-forkhead transcription factor complex [GO:0097221], TEAD-YAP complex [GO:0140552], GO:1990378, CSL-Notch-Mastermind transcription factor complex [GO:1990433], CLOCK-BMAL transcription complex [GO:1990513], ATF4-CREB1 transcription factor complex [GO:1990589], ATF1-ATF4 transcription factor complex [GO:1990590], CHOP-ATF4 complex [GO:1990617], C/EBP complex [GO:1990647], Nkx-2.5 complex [GO:1990664], beta-catenin-TCF complex [GO:1990907]